{
  "gene": "UniProtKB:Q8TDX6",
  "term_id": "GO:0050650",
  "gene_name": "Chondroitin sulfate N-acetylgalactosaminyltransferase 1",
  "gene_symbol": "CSGALNACT1",
  "term_label": "chondroitin sulfate proteoglycan biosynthetic process"
}